regulation of ectodermal cell fate specification [GO:0042665] (biological process) Also known as: regulation of ectoderm cell fate specification Sources: GOC:go_curators Subtypes: negative regulation of ectodermal cell fate specification [GO:0042666] Relationships: is a type of regulation of cell fate specification [GO:0042659]; regulates ectodermal cell fate specification [GO:0001715] Definition: Any process that mediates the specification of a cell into an ectoderm cell.